{
  "gene_name": "Corneodesmosin",
  "term_id": "GO:0042803",
  "gene_symbol": "CDSN",
  "term_label": "protein homodimerization activity",
  "gene": "UniProtKB:Q15517"
}